methylthioalkylmalate synthase activity [GO:0010177] (molecular function) Relationships: is a type of acyltransferase activity, acyl groups converted into alkyl on transfer [GO:0046912] Definition: Catalysis of the reaction: acetyl-CoA + an omega-(methylsulfanyl)-2-oxoalkanoate + H2O = a 2-(omega-methylsulfanyl)alkylmalate + CoA + H+. Sources: RHEA:50624 Also known as: 2-(2'-methylthio)ethylmalate synthase activity